{
  "gene": "UniProtKB:Q8IWV7",
  "gene_name": "E3 ubiquitin-protein ligase UBR1",
  "term_label": "ubiquitin protein ligase activity",
  "term_id": "GO:0061630",
  "gene_symbol": "UBR1"
}